{
  "gene": "UniProtKB:A6NNZ2",
  "term_label": "microtubule",
  "gene_symbol": "TUBB8B",
  "term_id": "GO:0005874",
  "gene_name": "Tubulin beta 8B"
}